{
  "term_label": "toll-like receptor signaling pathway",
  "term_id": "GO:0002224",
  "gene_symbol": "MAPKAPK2",
  "gene_name": "MAP kinase-activated protein kinase 2",
  "gene": "UniProtKB:P49137"
}